negative regulation of L-glutamate import across plasma membrane [GO:0002037] (biological process) Relationships: is a type of regulation of L-glutamate import across plasma membrane [GO:0002036]; is_a negative regulation of organic acid transport [GO:0032891]; is a type of negative regulation of transmembrane transport [GO:0034763]; is a type of negative regulation of amino acid transport [GO:0051956]; negatively regulates L-glutamate import across plasma membrane [GO:0098712] Definition: Any process that stops, prevents or reduces the frequency, rate or extent of L-glutamate import into a cell. Subtypes: GO:0051948 Sources: GOC:TermGenie Also known as: down regulation of L-glutamate transport, down-regulation of L-glutamate transport, downregulation of L-glutamate transport, negative regulation of L-glutamate import, negative regulation of L-glutamate transport, regulation of L-glutamate import, down regulation of L-glutamate import, down-regulation of L-glutamate import, downregulation of L-glutamate import, inhibition of L-glutamate import, inhibition of L-glutamate transport, inhibition of L-glutamate uptake, down regulation of L-glutamate uptake, down-regulation of L-glutamate uptake, downregulation of L-glutamate uptake, negative regulation of L-glutamate uptake